{
  "term_id": "GO:0042288",
  "term_label": "MHC class I protein binding",
  "gene_name": "Paired immunoglobulin-like type 2 receptor beta",
  "gene_symbol": "PILRB",
  "gene": "UniProtKB:Q9UKJ0"
}